{
  "term_id": "GO:0030154",
  "gene": "UniProtKB:O14627",
  "gene_name": "Homeobox protein CDX-4",
  "term_label": "cell differentiation",
  "gene_symbol": "CDX4"
}